{
  "gene": "UniProtKB:P04798",
  "gene_name": "Cytochrome P450 1A1",
  "gene_symbol": "CYP1A1",
  "term_id": "GO:0042178",
  "term_label": "xenobiotic catabolic process"
}